{
  "gene": "UniProtKB:Q96IK5",
  "term_id": "GO:0005634",
  "term_label": "nucleus",
  "gene_name": "Germ cell-less protein-like 1",
  "gene_symbol": "GMCL1"
}